{
  "term_id": "GO:0005829",
  "term_label": "cytosol",
  "gene_name": "Syncoilin",
  "gene_symbol": "SYNC",
  "gene": "UniProtKB:Q9H7C4"
}